{
  "gene": "UniProtKB:Q0VG06",
  "term_id": "UNKNOWN:0001",
  "gene_name": "Fanconi anemia core complex-associated protein 100",
  "gene_symbol": "FAAP100",
  "term_label": "Unknown molecular function"
}